{
  "gene_symbol": "CYP3A43",
  "gene_name": "Cytochrome P450 3A43",
  "term_id": "GO:0101020",
  "term_label": "estrogen 16-alpha-hydroxylase activity",
  "gene": "UniProtKB:Q9HB55"
}